{
  "gene": "UniProtKB:Q8NH70",
  "gene_name": "Olfactory receptor 4A16",
  "term_label": "olfactory receptor activity",
  "term_id": "GO:0004984",
  "gene_symbol": "OR4A16"
}